{
  "gene_name": "Transcription factor E2F6",
  "gene_symbol": "E2F6",
  "term_label": "RNA polymerase II cis-regulatory region sequence-specific DNA binding",
  "gene": "UniProtKB:O75461",
  "term_id": "GO:0000978"
}